{
  "gene_name": "Cytoplasmic aconitate hydratase",
  "term_id": "GO:0003994",
  "gene": "UniProtKB:P21399",
  "term_label": "aconitate hydratase activity",
  "gene_symbol": "ACO1"
}